{
  "term_label": "Unknown cellular component",
  "gene_symbol": "SPDYE2",
  "gene": "UniProtKB:Q495Y8",
  "gene_name": "Speedy protein E2",
  "term_id": "UNKNOWN:0003"
}